{
  "gene": "UniProtKB:A8MUH7",
  "gene_name": "Putative PDZ domain-containing protein PDZK1P1",
  "gene_symbol": "PDZK1P1",
  "term_id": "GO:0005102",
  "term_label": "signaling receptor binding"
}